{
  "term_label": "antigen processing and presentation of endogenous peptide antigen via MHC class Ib",
  "gene_symbol": "ULBP3",
  "gene_name": "UL16-binding protein 3",
  "gene": "UniProtKB:Q9BZM4",
  "term_id": "GO:0002476"
}